{
  "term_id": "GO:0005737",
  "term_label": "cytoplasm",
  "gene_symbol": "NCF1C",
  "gene": "UniProtKB:A8MVU1",
  "gene_name": "Putative neutrophil cytosol factor 1C"
}